{
  "term_label": "SNAP receptor activity",
  "gene_symbol": "VAMP2",
  "term_id": "GO:0005484",
  "gene_name": "Vesicle-associated membrane protein 2",
  "gene": "UniProtKB:P63027"
}